{
  "gene": "UniProtKB:P05387",
  "term_id": "UNKNOWN:0003",
  "gene_symbol": "RPLP2",
  "gene_name": "Large ribosomal subunit protein P2",
  "term_label": "Unknown cellular component"
}